{
  "gene_name": "Probable G-protein coupled receptor 142",
  "term_id": "GO:0005886",
  "term_label": "plasma membrane",
  "gene_symbol": "GPR142",
  "gene": "UniProtKB:Q7Z601"
}